{
  "gene_symbol": "PF4",
  "gene": "UniProtKB:P02776",
  "gene_name": "Platelet factor 4",
  "term_id": "GO:0045236",
  "term_label": "CXCR chemokine receptor binding"
}